endobrevin-synaptobrevin 2-alpha-SNAP-NSF-syntaxin-4 complex [GO:0070766] (cellular component) Also known as: SNARE complex (Stx4, Napa, Vamp3, Nsf, Vamp2), Stx4-Napa-Vamp3-Nsf-Vamp2 complex Relationships: is a type of SNARE complex [GO:0031201] Definition: A SNARE complex that contains endobrevin (VAMP8), synaptobrevin 2 (VAMP2), alpha-SNAP, NSF, and syntaxin 4 (or orthologs thereof). References: PMID:8973549